{
  "term_id": "GO:0042626",
  "gene_name": "Phosphatidylcholine translocator ABCB4",
  "gene": "UniProtKB:P21439",
  "term_label": "ATPase-coupled transmembrane transporter activity",
  "gene_symbol": "ABCB4"
}